{
  "gene": "UniProtKB:Q96G97",
  "term_label": "Unknown molecular function",
  "gene_name": "Seipin",
  "term_id": "UNKNOWN:0001",
  "gene_symbol": "BSCL2"
}